{
  "term_id": "GO:0051726",
  "gene_symbol": "JUNB",
  "term_label": "regulation of cell cycle",
  "gene": "UniProtKB:P17275",
  "gene_name": "Transcription factor JunB"
}